{
  "term_label": "Unknown cellular component",
  "gene_symbol": "FRA10AC1",
  "term_id": "UNKNOWN:0003",
  "gene": "UniProtKB:Q70Z53",
  "gene_name": "Protein FRA10AC1"
}